{
  "gene_name": "4-aminobutyrate aminotransferase, mitochondrial",
  "term_label": "mitochondrion",
  "gene_symbol": "ABAT",
  "gene": "UniProtKB:P80404",
  "term_id": "GO:0005739"
}